{
  "term_id": "GO:0071039",
  "gene_name": "Zinc finger CCHC domain-containing protein 7",
  "term_label": "nuclear polyadenylation-dependent CUT catabolic process",
  "gene": "UniProtKB:Q8N3Z6",
  "gene_symbol": "ZCCHC7"
}